regulation of relaxation of smooth muscle [GO:1901080] (biological process) Definition: Any process that modulates the frequency, rate or extent of relaxation of smooth muscle. Sources: GOC:TermGenie Also known as: regulation of smooth muscle relaxation Relationships: is a type of regulation of relaxation of muscle [GO:1901077]; regulates relaxation of smooth muscle [GO:0044557] Subtypes: regulation of uterine smooth muscle relaxation [GO:1900719], negative regulation of relaxation of smooth muscle [GO:1901081], positive regulation of relaxation of smooth muscle [GO:1901082]